{
  "term_id": "UNKNOWN:0002",
  "gene": "UniProtKB:Q8IY51",
  "term_label": "Unknown biological process",
  "gene_symbol": "TIGD4",
  "gene_name": "Tigger transposable element-derived protein 4"
}